{
  "term_id": "GO:0045944",
  "gene": "UniProtKB:P05549",
  "gene_name": "Transcription factor AP-2-alpha",
  "term_label": "positive regulation of transcription by RNA polymerase II",
  "gene_symbol": "TFAP2A"
}